{
  "term_label": "Rho protein signal transduction",
  "gene_symbol": "EPS8L2",
  "gene": "UniProtKB:Q9H6S3",
  "term_id": "GO:0007266",
  "gene_name": "Epidermal growth factor receptor kinase substrate 8-like protein 2"
}